{
  "gene": "UniProtKB:A0A0B4J274",
  "term_label": "response to bacterium",
  "gene_name": "T cell receptor alpha variable 20",
  "term_id": "GO:0009617",
  "gene_symbol": "TRAV20"
}